{
  "term_id": "GO:0042632",
  "gene": "UniProtKB:P16233",
  "gene_symbol": "PNLIP",
  "gene_name": "Pancreatic triacylglycerol lipase",
  "term_label": "cholesterol homeostasis"
}